regulation of immune response [GO:0050776] (biological process) Sources: GOC:ai Definition: Any process that modulates the frequency, rate or extent of the immune response, the immunological reaction of an organism to an immunogenic stimulus. Relationships: is a type of GO:0002682; is a type of regulation of response to stimulus [GO:0048583]; regulates immune response [GO:0006955] Subtypes: immune response-regulating signaling pathway [GO:0002764], GO:0002819, regulation of type 2 immune response [GO:0002828], regulation of immune response to tumor cell [GO:0002837], regulation of inflammatory response to antigenic stimulus [GO:0002861], regulation of humoral immune response [GO:0002920], GO:0032820, regulation of CD4-positive, CD25-positive, alpha-beta regulatory T cell differentiation involved in immune response [GO:0032832], regulation of mast cell activation involved in immune response [GO:0033006], regulation of eosinophil degranulation [GO:0043309], regulation of neutrophil degranulation [GO:0043313], regulation of memory T cell differentiation [GO:0043380], regulation of innate immune response [GO:0045088], regulation of T-helper cell differentiation [GO:0045622], negative regulation of immune response [GO:0050777], GO:0050778, GO:0050854, regulation of Fc receptor mediated stimulatory signaling pathway [GO:0060368], regulation of plasma cell differentiation [GO:1900098], regulation of basophil degranulation [GO:1903581], regulation of T cell activation via T cell receptor contact with antigen bound to MHC molecule on antigen presenting cell [GO:2001188], regulation of gamma-delta T cell activation involved in immune response [GO:2001191]